{
  "gene_name": "Galectin-9C",
  "gene_symbol": "LGALS9C",
  "term_id": "GO:0005829",
  "gene": "UniProtKB:Q6DKI2",
  "term_label": "cytosol"
}